UDP-arabinose 4-epimerase activity [GO:0050373] (molecular function) Also known as: UDP-D-xylose-4-epimerase activity, UDP arabinose epimerase activity, UDP-D-xylose 4-epimerase activity, UDP-L-arabinose 4-epimerase activity, UDParabinose 4-epimerase activity, uridine 5'-diphosphate-D-xylose 4-epimerase activity, uridine diphosphoarabinose epimerase activity Definition: Catalysis of the reaction: UDP-L-arabinose = UDP-alpha-D-xylose. Relationships: is a type of racemase and epimerase activity, acting on carbohydrates and derivatives [GO:0016857] Sources: EC:5.1.3.5, RHEA:11320